{
  "term_id": "UNKNOWN:0001",
  "gene_name": "26S proteasome non-ATPase regulatory subunit 3",
  "term_label": "Unknown molecular function",
  "gene": "UniProtKB:O43242",
  "gene_symbol": "PSMD3"
}